regulation of 1-phosphatidyl-1D-myo-inositol 4,5-bisphosphate biosynthetic process [GO:1902646] (biological process) Relationships: is_a GO:0010511; regulates 1-phosphatidyl-1D-myo-inositol 4,5-bisphosphate biosynthetic process [GO:1902635] Also known as: regulation of 1-phosphatidyl-1D-myo-inositol 4,5-bisphosphate anabolism, regulation of 1-phosphatidyl-1D-myo-inositol 4,5-bisphosphate biosynthesis, regulation of 1-phosphatidyl-1D-myo-inositol 4,5-bisphosphate formation, regulation of 1-phosphatidyl-1D-myo-inositol 4,5-bisphosphate synthesis References: PMID:22562153 Sources: GOC:TermGenie, GOC:di, GO_REF:0000058 Definition: Any process that modulates the frequency, rate or extent of 1-phosphatidyl-1D-myo-inositol 4,5-bisphosphate biosynthetic process. Subtypes: GO:1902647, positive regulation of 1-phosphatidyl-1D-myo-inositol 4,5-bisphosphate biosynthetic process [GO:1902648]